{
  "gene": "UniProtKB:O60478",
  "gene_symbol": "GPR137B",
  "term_id": "GO:0045671",
  "gene_name": "Integral membrane protein GPR137B",
  "term_label": "negative regulation of osteoclast differentiation"
}